{
  "term_label": "ubiquitin protein ligase activity",
  "gene_name": "Apoptosis-resistant E3 ubiquitin protein ligase 1",
  "term_id": "GO:0061630",
  "gene": "UniProtKB:O15033",
  "gene_symbol": "AREL1"
}